{
  "gene_symbol": "CBLN3",
  "term_label": "extracellular space",
  "term_id": "GO:0005615",
  "gene": "UniProtKB:Q6UW01",
  "gene_name": "Cerebellin-3"
}